{
  "gene_name": "NANOG neighbor homeobox",
  "gene_symbol": "NANOGNB",
  "gene": "UniProtKB:Q7Z5D8",
  "term_label": "Unknown biological process",
  "term_id": "UNKNOWN:0002"
}